CARD8 inflammasome complex assembly [GO:0140633] (biological process) Definition: The aggregation, arrangement and bonding together of a set of components to form a CARD8 inflammasome complex. Relationships: is a type of canonical inflammasome complex assembly [GO:0140632] References: PMID:33420028, PMID:33420033, PMID:33542150